{
  "gene_symbol": "ZNF701",
  "gene_name": "Zinc finger protein 701",
  "term_id": "GO:0005634",
  "term_label": "nucleus",
  "gene": "UniProtKB:Q9NV72"
}